RNA polymerase IV complex [GO:0000418] (cellular component) References: PMID:15692015, PMID:15766525, PMID:16140984, PMID:19110459 Sources: GOC:krc, GOC:mtg_sensu Relationships: is a type of DNA-directed RNA polymerase complex [GO:0000428]; is a type of GO:0140513 Definition: RNA polymerase IV is a multisubunit RNA polymerase complex found in the nucleus of plants and involved in accumulation of siRNAs and in DNA methylation-dependent silencing of endogenous repeated sequences. Pol IV is composed of subunits that are paralogous or identical to the 12 subunits of Pol II. The largest and second-largest subunits of Pol IV are the catalytic subunits and share similarity with the corresponding subunits of other eukaryotic and bacterial multisubunit RNA polymerases. The second largest subunit is also found in RNA polymerase V, while the largest subunit is found only in RNAP IV complex. Also known as: DNA-directed RNA polymerase IV complex, DNA-directed RNA polymerase IVa complex